{
  "gene": "UniProtKB:O95359",
  "term_label": "cerebral cortex development",
  "gene_symbol": "TACC2",
  "gene_name": "Transforming acidic coiled-coil-containing protein 2",
  "term_id": "GO:0021987"
}